{
  "gene_name": "Sorbitol dehydrogenase",
  "gene": "UniProtKB:Q00796",
  "gene_symbol": "SORD",
  "term_label": "L-iditol 2-dehydrogenase (NAD+) activity",
  "term_id": "GO:0003939"
}